synaptonemal complex [GO:0000795] (cellular component) Sources: DOI:10.5772/29752, GOC:elh Relationships: is a type of synaptonemal structure [GO:0099086] Definition: A proteinaceous scaffold found between homologous chromosomes during meiosis. It consists of 2 lateral elements and a central element, all running parallel to each other. Transverse filaments connect the lateral elements to the central element.